L-amino-acid N-acetyltransferase activity [GO:0140085] (molecular function) Definition: Catalysis of the reaction: acetyl-CoA + a L-amino acid = CoA + an N-acetyl-L-amino-acid. In some cases acetyl phosphate can be used as a donor. Sources: GOC:pg, RHEA:83863 Relationships: is a type of N-acetyltransferase activity [GO:0008080] Subtypes: L-glutamate N-acetyltransferase activity [GO:0004042], GO:0004358, L-lysine N-acetyltransferase activity, acting on acetyl phosphate as donor [GO:0004468], L-aspartate N-acetyltransferase activity [GO:0017188], L-cysteine-S-conjugate N-acetyltransferase activity [GO:0047198], L-histidine N-acetyltransferase activity [GO:0047981], GO:0050050, L-phenylalanine N-acetyltransferase activity [GO:0050176], L-lysine N6-acetyltransferase [GO:0090595], L-methionine N-acyltransferase activity [GO:0103045]